substance P secretion, neurotransmission [GO:1990793] (biological process) Regulation: regulated by regulation of substance P secretion, neurotransmission [GO:1904494]; negatively regulated by negative regulation of substance P secretion, neurotransmission [GO:1904495]; positively regulated by positive regulation of substance P secretion, neurotransmission [GO:1904496] Relationships: is a type of neurotransmitter secretion [GO:0007269]; is_a substance P secretion [GO:1990772] References: PMID:15292051 Definition: The controlled release of substance P by a cell, in which the substance P acts as a neurotransmitter.